monocarboxylic acid transmembrane transporter activity [GO:0008028] (molecular function) Also known as: monocarboxylate carrier, prostaglandin/thromboxane transporter activity Definition: Enables the transfer of monocarboxylic acids from one side of a membrane to the other. A monocarboxylic acid is an organic acid with one COOH group. Relationships: is a type of carboxylic acid transmembrane transporter activity [GO:0046943]; is part of monocarboxylic acid transport [GO:0015718] Sources: GOC:ai Subtypes: GO:0015123, bile acid transmembrane transporter activity [GO:0015125], lactate transmembrane transporter activity [GO:0015129], GO:0015133, GO:0015185, biotin transmembrane transporter activity [GO:0015225], fatty acid transmembrane transporter activity [GO:0015245], secondary active monocarboxylate transmembrane transporter activity [GO:0015355], formate transmembrane transporter activity [GO:0015499], shikimate transmembrane transporter activity [GO:0015530], GO:0015568, ATPase-coupled monocarboxylic acid transmembrane transporter activity [GO:0033285], L-hydroxyproline transmembrane transporter activity [GO:0034590], D-galactonate transmembrane transporter activity [GO:0042881], 3-hydroxyphenylpropionic acid transmembrane transporter activity [GO:0042926], chrysobactin transmembrane transporter activity [GO:0042933], GO:0043879, pyruvate transmembrane transporter activity [GO:0050833], phosphoenolpyruvate transmembrane transporter activity [GO:0089721], nicotinate transmembrane transporter activity [GO:0090416], abscisic acid transmembrane transporter activity [GO:0090440], GO:0140485, 4-hydroxyphenylacetate transmembrane transporter activity [GO:1901241], dethiobiotin transmembrane transporter activity [GO:1901604], glycerate transmembrane transporter activity [GO:1901974]